{
  "gene_symbol": "DNMT3L",
  "gene": "UniProtKB:Q9UJW3",
  "term_label": "enzyme activator activity",
  "gene_name": "DNA (cytosine-5)-methyltransferase 3-like",
  "term_id": "GO:0008047"
}